{
  "term_label": "plasma membrane",
  "gene": "UniProtKB:P11230",
  "term_id": "GO:0005886",
  "gene_name": "Acetylcholine receptor subunit beta",
  "gene_symbol": "CHRNB1"
}